{
  "term_label": "RNA polymerase II cis-regulatory region sequence-specific DNA binding",
  "gene_name": "Transcriptional activator Myb",
  "gene": "UniProtKB:P10242",
  "gene_symbol": "MYB",
  "term_id": "GO:0000978"
}